{
  "gene_symbol": "TMEM263",
  "term_label": "Unknown cellular component",
  "term_id": "UNKNOWN:0003",
  "gene": "UniProtKB:Q8WUH6",
  "gene_name": "Transmembrane protein 263"
}